{
  "gene_symbol": "SLC2A2",
  "gene": "UniProtKB:P11168",
  "term_label": "dehydroascorbic acid transport",
  "gene_name": "Solute carrier family 2, facilitated glucose transporter member 2",
  "term_id": "GO:0070837"
}